{
  "gene": "UniProtKB:Q9H2K8",
  "term_id": "GO:0048812",
  "term_label": "neuron projection morphogenesis",
  "gene_symbol": "TAOK3",
  "gene_name": "Serine_threonine-protein kinase TAO3"
}